hydrogenosome [GO:0042566] (cellular component) Definition: A spherical, membrane-bounded organelle found in some anaerobic protozoa, which participates in ATP and molecular hydrogen formation. References: PMID:11197234, PMID:11293569 Sources: GOC:jl Relationships: is a type of intracellular membrane-bounded organelle [GO:0043231]; is part of GO:0005737